{
  "term_label": "sodium-independent organic anion transport",
  "gene_symbol": "SLCO1A2",
  "gene_name": "Solute carrier organic anion transporter family member 1A2",
  "term_id": "GO:0043252",
  "gene": "UniProtKB:P46721"
}